{
  "term_label": "Unknown biological process",
  "gene_symbol": "HDLBP",
  "term_id": "UNKNOWN:0002",
  "gene": "UniProtKB:Q00341",
  "gene_name": "Vigilin"
}